{
  "term_id": "GO:0003779",
  "gene": "UniProtKB:Q8IVE3",
  "gene_symbol": "PLEKHH2",
  "term_label": "actin binding",
  "gene_name": "Pleckstrin homology domain-containing family H member 2"
}